multicellular organism adhesion to substrate [GO:0022609] (biological process) Sources: GOC:isa_complete Subtypes: puparial adhesion [GO:0007594] Definition: The attachment of a multicellular organism to a surface or material. Relationships: is a type of GO:0022608